{
  "gene": "UniProtKB:Q9UD57",
  "gene_symbol": "NKX1-2",
  "gene_name": "NK1 transcription factor-related protein 2",
  "term_id": "GO:0006357",
  "term_label": "regulation of transcription by RNA polymerase II"
}